{
  "term_label": "nucleolus",
  "gene_symbol": "SURF6",
  "gene": "UniProtKB:O75683",
  "term_id": "GO:0005730",
  "gene_name": "Surfeit locus protein 6"
}